{
  "gene": "UniProtKB:Q9UKJ1",
  "term_label": "Unknown cellular component",
  "gene_name": "Paired immunoglobulin-like type 2 receptor alpha",
  "gene_symbol": "PILRA",
  "term_id": "UNKNOWN:0003"
}